{
  "term_label": "hormone activity",
  "gene_symbol": "CGB7",
  "gene": "UniProtKB:P0DN87",
  "term_id": "GO:0005179",
  "gene_name": "Choriogonadotropin subunit beta 7"
}